{
  "gene_name": "E3 ubiquitin-protein ligase RNF14",
  "gene_symbol": "RNF14",
  "gene": "UniProtKB:Q9UBS8",
  "term_id": "GO:0000151",
  "term_label": "ubiquitin ligase complex"
}